{
  "term_label": "synapse",
  "gene_name": "PI-PLC X domain-containing protein 3",
  "gene": "UniProtKB:Q63HM9",
  "gene_symbol": "PLCXD3",
  "term_id": "GO:0045202"
}